nitrate catabolic process [GO:0043602] (BP) Sources: GOC:jl Also known as: nitrate disassimilation, nitrate dissimilation Definition: The chemical reactions and pathways resulting in the breakdown of nitrates, inorganic or organic salts and esters of nitric acid. Relationships: is_a catabolic process [GO:0009056]; is a type of nitrate metabolic process [GO:0042126]